{
  "gene_symbol": "NR2F2",
  "gene_name": "COUP transcription factor 2",
  "term_id": "GO:0004879",
  "gene": "UniProtKB:P24468",
  "term_label": "nuclear receptor activity"
}